{
  "gene": "UniProtKB:P01911",
  "gene_symbol": "HLA-DRB1",
  "term_id": "GO:0019886",
  "gene_name": "HLA class II histocompatibility antigen, DRB1 beta chain",
  "term_label": "antigen processing and presentation of exogenous peptide antigen via MHC class II"
}